{
  "gene_name": "Interleukin-1 receptor-associated kinase-like 2",
  "gene": "UniProtKB:O43187",
  "term_label": "interleukin-1-mediated signaling pathway",
  "gene_symbol": "IRAK2",
  "term_id": "GO:0070498"
}